positive regulation of corticosteroid hormone secretion [GO:2000848] (biological process) Relationships: is a type of GO:2000833; is a type of regulation of corticosteroid hormone secretion [GO:2000846]; positively regulates corticosteroid hormone secretion [GO:0035930] Definition: Any process that activates or increases the frequency, rate or extent of corticosteroid hormone secretion. Also known as: positive regulation of corticosteroid secretion Sources: GOC:sl Subtypes: GO:2000851, positive regulation of mineralocorticoid secretion [GO:2000857]